{
  "term_label": "nuclear speck",
  "gene_symbol": "SNURFL",
  "gene_name": "Putative SNURF-like protein",
  "gene": "UniProtKB:B1AK76",
  "term_id": "GO:0016607"
}